{
  "gene_symbol": "GATM",
  "term_label": "creatine biosynthetic process",
  "term_id": "GO:0006601",
  "gene": "UniProtKB:P50440",
  "gene_name": "Glycine amidinotransferase, mitochondrial"
}